sulfate:proton symporter activity [GO:0008512] (molecular function) Relationships: is a type of secondary active sulfate transmembrane transporter activity [GO:0008271]; is a type of GO:0015295 Sources: TC:2.A.53.-.- Subtypes: high-affinity sulfate:proton symporter activity [GO:0009675], GO:0009676 Definition: Enables the transfer of a solute or solutes from one side of a membrane to the other according to the reaction: sulfate(out) + H+(out) = sulfate(in) + H+(in). Also known as: sulfate/hydrogen symporter activity, sulfate:hydrogen symporter activity, sulphate:hydrogen symporter activity